{
  "term_id": "GO:0015721",
  "term_label": "bile acid and bile salt transport",
  "gene_symbol": "SLC10A1",
  "gene_name": "Hepatic sodium_bile acid cotransporter",
  "gene": "UniProtKB:Q14973"
}